{
  "term_id": "UNKNOWN:0002",
  "gene": "UniProtKB:Q9BYD9",
  "gene_symbol": "ACTRT3",
  "term_label": "Unknown biological process",
  "gene_name": "Actin-related protein T3"
}